{
  "gene": "UniProtKB:Q6ISB3",
  "term_label": "DNA-binding transcription activator activity, RNA polymerase II-specific",
  "term_id": "GO:0001228",
  "gene_name": "Grainyhead-like protein 2 homolog",
  "gene_symbol": "GRHL2"
}